{
  "term_label": "chromatin organization",
  "gene_name": "Transcription intermediary factor 1-beta",
  "gene": "UniProtKB:Q13263",
  "term_id": "GO:0006325",
  "gene_symbol": "TRIM28"
}